{
  "gene": "UniProtKB:Q9Y3B3",
  "term_id": "GO:0005783",
  "gene_name": "Transmembrane emp24 domain-containing protein 7",
  "gene_symbol": "TMED7",
  "term_label": "endoplasmic reticulum"
}